{
  "term_label": "ATP hydrolysis activity",
  "gene_name": "Putative endoplasmin-like protein",
  "gene_symbol": "HSP90B2P",
  "term_id": "GO:0016887",
  "gene": "UniProtKB:Q58FF3"
}